{
  "gene_name": "Dual specificity mitogen-activated protein kinase kinase 3",
  "term_label": "MAPK cascade",
  "gene_symbol": "MAP2K3",
  "gene": "UniProtKB:P46734",
  "term_id": "GO:0000165"
}